{
  "term_label": "keratin filament",
  "gene": "UniProtKB:P12035",
  "term_id": "GO:0045095",
  "gene_name": "Keratin, type II cytoskeletal 3",
  "gene_symbol": "KRT3"
}